{
  "term_label": "tail-anchored membrane protein insertion into ER membrane",
  "gene_name": "Guided entry of tail-anchored proteins factor 1",
  "gene_symbol": "GET1",
  "gene": "UniProtKB:O00258",
  "term_id": "GO:0071816"
}